{
  "term_label": "Unknown molecular function",
  "gene_symbol": "KIAA0040",
  "gene_name": "Uncharacterized protein KIAA0040",
  "gene": "UniProtKB:Q15053",
  "term_id": "UNKNOWN:0001"
}